neural crest cell development [GO:0014032] (biological process) Definition: The process aimed at the progression of a neural crest cell over time, from initial commitment of the cell to its specific fate, to the fully functional differentiated cell. Relationships: is a type of stem cell development [GO:0048864]; is part of neural crest cell differentiation [GO:0014033] Subtypes: cardiac neural crest cell development involved in heart development [GO:0061308] Sources: GOC:dh, GOC:ef